trans spliceosomal complex [GO:0071023] (cellular component) Relationships: is a type of GO:0005681; has part U5 snRNP [GO:0005682]; has part U2 snRNP [GO:0005686]; has part GO:0005687; has part U6 snRNP [GO:0005688]; has part SL snRNP [GO:0071024] Definition: A spliceosomal complex that forms during the addition of a specific spliced leader (SL) sequence to the 5'-end of a messenger RNA primary transcript, a process which occurs in a number of eukaryotic organisms, including trypanosomatid protozoans, euglenoids, nematodes, trematodes, and chordates. Sources: GOC:krc, ISBN:0879697393